{
  "gene_name": "Endogenous retrovirus group K member 11 Pol protein",
  "term_label": "Unknown cellular component",
  "gene_symbol": "ERVK-11",
  "term_id": "UNKNOWN:0003",
  "gene": "UniProtKB:Q9UQG0"
}